{
  "term_label": "cysteine-type endopeptidase activity",
  "gene_name": "Cathepsin O",
  "gene_symbol": "CTSO",
  "gene": "UniProtKB:P43234",
  "term_id": "GO:0004197"
}